{
  "term_id": "GO:0032007",
  "gene_symbol": "TNFAIP8L1",
  "term_label": "negative regulation of TOR signaling",
  "gene_name": "Tumor necrosis factor alpha-induced protein 8-like protein 1",
  "gene": "UniProtKB:Q8WVP5"
}